{
  "gene_name": "Trefoil factor 3",
  "term_label": "extracellular space",
  "gene": "UniProtKB:Q07654",
  "term_id": "GO:0005615",
  "gene_symbol": "TFF3"
}